P-type sodium:potassium-exchanging transporter activity involved in regulation of cardiac muscle cell membrane potential [GO:0086037] (molecular function) Relationships: is a type of P-type sodium:potassium-exchanging transporter activity [GO:0005391]; is part of regulation of cardiac muscle cell membrane potential [GO:0086036] Definition: Enables the transfer of a solute or solutes from one side of a membrane to the other according to the reaction: ATP + H2O + Na+(in) + K+(out) = ADP + phosphate + Na+(out) + K+(in), that contributes to regulating the membrane potential of a cardiac muscle cell. Sources: GOC:BHF, GOC:mtg_cardiac_conduct_nov11